{
  "term_label": "alpha-N-acetylgalactosaminide alpha-2,6-sialyltransferase activity",
  "gene_symbol": "ST6GALNAC5",
  "gene_name": "Alpha-N-acetylgalactosaminide alpha-2,6-sialyltransferase 5",
  "term_id": "GO:0001665",
  "gene": "UniProtKB:Q9BVH7"
}